{
  "gene_symbol": "OPN3",
  "term_id": "GO:0005886",
  "term_label": "plasma membrane",
  "gene": "UniProtKB:Q9H1Y3",
  "gene_name": "Opsin-3"
}